phosphomannan mannosephosphotransferase activity [GO:0047361] (molecular function) Definition: Catalysis of the reaction: phosphomannan(n) + GDP-mannose = phosphomannan(n+1) + GMP. Also known as: GDP-mannose:phosphomannan mannose phosphotransferase activity Sources: EC:2.7.8.9, MetaCyc:2.7.8.9-RXN Relationships: is a type of phosphotransferase activity, for other substituted phosphate groups [GO:0016780]